{
  "gene_name": "Heat shock protein beta-2",
  "gene_symbol": "HSPB2",
  "term_id": "GO:0051082",
  "term_label": "unfolded protein binding",
  "gene": "UniProtKB:Q16082"
}